{
  "gene_symbol": "SLC4A9",
  "term_id": "GO:0015701",
  "term_label": "bicarbonate transport",
  "gene_name": "Anion exchange protein 4",
  "gene": "UniProtKB:Q96Q91"
}